negative regulation of ERAD pathway [GO:1904293] (biological process) Relationships: is_a negative regulation of proteasomal protein catabolic process [GO:1901799]; is a type of negative regulation of response to endoplasmic reticulum stress [GO:1903573]; is a type of regulation of ERAD pathway [GO:1904292]; negatively regulates ERAD pathway [GO:0036503] References: PMID:22590560 Sources: GOC:PARL, GOC:TermGenie, GOC:bf, GO_REF:0000058 Definition: Any process that stops, prevents or reduces the frequency, rate or extent of ERAD pathway. Also known as: down regulation of ERAD pathway, down regulation of endoplasmic reticulum-associated degradation, down-regulation of ERAD pathway, down-regulation of endoplasmic reticulum-associated degradation, downregulation of ERAD pathway, downregulation of endoplasmic reticulum-associated degradation, negative regulation of endoplasmic reticulum-associated degradation, inhibition of ERAD pathway, inhibition of endoplasmic reticulum-associated degradation, down regulation of ER-associated degradation pathway, down regulation of endoplasmic reticulum-associated protein degradation pathway, down-regulation of ER-associated degradation pathway, down-regulation of endoplasmic reticulum-associated protein degradation pathway, downregulation of ER-associated degradation pathway, downregulation of endoplasmic reticulum-associated protein degradation pathway, inhibition of ER-associated degradation pathway, inhibition of endoplasmic reticulum-associated protein degradation pathway, negative regulation of ER-associated degradation pathway, negative regulation of endoplasmic reticulum-associated protein degradation pathway